{
  "term_label": "microtubule",
  "gene_name": "Dynein regulatory complex subunit 4",
  "term_id": "GO:0005874",
  "gene": "UniProtKB:O95995",
  "gene_symbol": "GAS8"
}